{
  "gene": "UniProtKB:Q8NCX0",
  "term_id": "UNKNOWN:0001",
  "term_label": "Unknown molecular function",
  "gene_name": "Coiled-coil domain-containing protein 150",
  "gene_symbol": "CCDC150"
}